dGMP catabolic process [GO:0046055] (BP) Definition: The chemical reactions and pathways resulting in the breakdown of dGMP, deoxyguanosine monophosphate (2'-deoxyguanosine 5'-phosphate). Relationships: is a type of GO:0009155; is a type of purine deoxyribonucleoside monophosphate catabolic process [GO:0009172]; is a type of dGMP metabolic process [GO:0046054] Also known as: dGMP breakdown, dGMP catabolism, dGMP degradation Sources: GOC:go_curators